{
  "gene": "UniProtKB:Q15800",
  "term_id": "GO:0000254",
  "gene_symbol": "MSMO1",
  "gene_name": "Methylsterol monooxygenase 1",
  "term_label": "C-4 methylsterol oxidase activity"
}